benzaldehyde dehydrogenase (NAD+) activity [GO:0018479] (molecular function) Also known as: benzaldehyde (NAD) dehydrogenase activity, benzaldehyde:NAD+ oxidoreductase activity Relationships: is_a GO:0004029 Sources: EC:1.2.1.28 Definition: Catalysis of the reaction: benzaldehyde + NAD+ + H2O = benzoate + NADH + H+.